{
  "gene_symbol": "KIAA1755",
  "term_id": "GO:0005085",
  "gene": "UniProtKB:Q5JYT7",
  "gene_name": "Uncharacterized protein KIAA1755",
  "term_label": "guanyl-nucleotide exchange factor activity"
}